{
  "gene_symbol": "UBB",
  "term_label": "cytosolic ribosome",
  "gene": "UniProtKB:P0CG47",
  "term_id": "GO:0022626",
  "gene_name": "Polyubiquitin-B"
}